dentate gyrus development [GO:0021542] (BP) Relationships: is a type of anatomical structure development [GO:0048856]; BFO_0000050 hippocampus development [GO:0021766] Sources: GOC:cls, GOC:dgh, GOC:dph, GOC:jid, GO_REF:0000021 Definition: The process whose specific outcome is the progression of the dentate gyrus over time, from its formation to the mature structure. The dentate gyrus is one of two interlocking gyri of the hippocampus. It contains granule cells, which project to the pyramidal cells and interneurons of the CA3 region of the ammon gyrus.